{
  "term_label": "positive regulation of cytosolic calcium ion concentration",
  "gene": "UniProtKB:P51677",
  "gene_symbol": "CCR3",
  "term_id": "GO:0007204",
  "gene_name": "C-C chemokine receptor type 3"
}